endomitotic cell cycle [GO:0007113] (biological process) Definition: A mitotic cell cycle in which chromosomes are replicated and sister chromatids separate, but spindle formation, nuclear membrane breakdown and nuclear division do not occur, resulting in an increased number of chromosomes in the cell. Sources: GOC:curators, GOC:dos, GOC:expert_vm Also known as: endomitosis Note: Note that this term should not be confused with 'abortive mitotic cell cycle ; GO:0033277'. Although abortive mitosis is sometimes called endomitosis, GO:0033277 refers to a process in which a mitotic spindle forms and chromosome separation begins. Relationships: is a type of mitotic cell cycle [GO:0000278]